positive regulation of response to wounding [GO:1903036] (biological process) Subtypes: positive regulation of axon regeneration [GO:0048680], positive regulation of wound healing [GO:0090303], positive regulation of inflammatory response to wounding [GO:0106016] References: PMID:19164535 Sources: GOC:TermGenie, GOC:kmv, GO_REF:0000058 Definition: Any process that activates or increases the frequency, rate or extent of response to wounding. Also known as: positive regulation of physiological response to wounding, up regulation of physiological response to wounding, up regulation of response to wounding, up-regulation of physiological response to wounding, up-regulation of response to wounding, upregulation of physiological response to wounding, upregulation of response to wounding, activation of physiological response to wounding, activation of response to wounding Relationships: is a type of positive regulation of response to stimulus [GO:0048584]; is a type of regulation of response to wounding [GO:1903034]; positively regulates GO:0009611